negative regulation of hyaluronan biosynthetic process [GO:1900126] (biological process) Relationships: is a type of negative regulation of macromolecule biosynthetic process [GO:0010558]; is a type of negative regulation of carbohydrate metabolic process [GO:0045912]; is_a GO:1900125; negatively regulates hyaluronan biosynthetic process [GO:0030213] Definition: Any process that stops, prevents or reduces the frequency, rate or extent of hyaluronan biosynthetic process. Also known as: down regulation of hyaluronan anabolism, down regulation of hyaluronan biosynthesis, down regulation of hyaluronan biosynthetic process, down regulation of hyaluronan formation, down regulation of hyaluronan synthesis, down-regulation of hyaluronan anabolism, down-regulation of hyaluronan biosynthesis, down-regulation of hyaluronan biosynthetic process, down-regulation of hyaluronan formation, down-regulation of hyaluronan synthesis, downregulation of hyaluronan anabolism, downregulation of hyaluronan biosynthesis, downregulation of hyaluronan biosynthetic process, downregulation of hyaluronan formation, downregulation of hyaluronan synthesis, inhibition of hyaluronan anabolism, inhibition of hyaluronan biosynthesis, inhibition of hyaluronan formation, inhibition of hyaluronan synthesis, negative regulation of hyaluronan anabolism, negative regulation of hyaluronan biosynthesis, negative regulation of hyaluronan formation, negative regulation of hyaluronan synthesis, inhibition of hyaluronan biosynthetic process Sources: GOC:TermGenie, GOC:yaf